{
  "gene_symbol": "C2orf83",
  "gene": "UniProtKB:Q53S99",
  "term_id": "UNKNOWN:0002",
  "gene_name": "Folate transporter-like protein C2orf83",
  "term_label": "Unknown biological process"
}